{
  "gene_symbol": "RAB20",
  "term_label": "plasma membrane",
  "gene_name": "Ras-related protein Rab-20",
  "gene": "UniProtKB:Q9NX57",
  "term_id": "GO:0005886"
}